{
  "gene_name": "Ly6_PLAUR domain-containing protein 8",
  "gene": "UniProtKB:Q6UX82",
  "gene_symbol": "LYPD8",
  "term_id": "GO:0005615",
  "term_label": "extracellular space"
}